{
  "gene": "UniProtKB:Q08999",
  "term_id": "GO:0000785",
  "gene_symbol": "RBL2",
  "gene_name": "Retinoblastoma-like protein 2",
  "term_label": "chromatin"
}